negative regulation of protein oxidation [GO:1904807] (biological process) Definition: Any process that stops, prevents or reduces the frequency, rate or extent of protein oxidation. Relationships: is_a GO:0031400; is a type of regulation of protein oxidation [GO:1904806]; negatively regulates GO:0018158 Also known as: down regulation of protein amino acid oxidation, down regulation of protein oxidation, down-regulation of protein amino acid oxidation, down-regulation of protein oxidation, downregulation of protein amino acid oxidation, downregulation of protein oxidation, negative regulation of protein amino acid oxidation, inhibition of protein amino acid oxidation, inhibition of protein oxidation References: PMID:22719267 Sources: GOC:TermGenie, GO_REF:0000058